4-(dimethylamino)phenylazoxybenzene reductase activity [GO:0047136] (molecular function) Sources: EC:1.7.1.11, RHEA:19789 Relationships: is a type of oxidoreductase activity, acting on other nitrogenous compounds as donors, with NAD or NADP as acceptor [GO:0046857] Also known as: 4-(dimethylamino)phenylazobenzene:NADP+ oxidoreductase activity, N,N-dimethyl-p-aminoazobenzene oxide reductase activity, NADPH-dependent DMAB N-oxide reductase activity, NADPH2:4-(dimethylamino)phenylazoxybenzene oxidoreductase activity, NADPH:4-(dimethylamino)phenylazoxybenzene oxidoreductase activity, dimethylaminoazobenzene N-oxide reductase activity Definition: Catalysis of the reaction: 4-(dimethylamino)azobenzene + H2O + NADP+ = 4-(dimethylamino)phenylazoxybenzene + H+ + NADPH.